{
  "term_id": "GO:0004999",
  "term_label": "vasoactive intestinal polypeptide receptor activity",
  "gene_symbol": "VIPR2",
  "gene": "UniProtKB:P41587",
  "gene_name": "Vasoactive intestinal polypeptide receptor 2"
}